{
  "gene_name": "MyoD family inhibitor domain-containing protein",
  "term_id": "GO:0046328",
  "term_label": "regulation of JNK cascade",
  "gene_symbol": "MDFIC",
  "gene": "UniProtKB:Q9P1T7"
}